prostaglandin receptor internalization [GO:1990767] (biological process) Relationships: is a type of G protein-coupled receptor internalization [GO:0002031] Definition: The process that results in the uptake of a prostaglandin receptor into an endocytic vesicle. References: PMID:15937517